T-helper 2 cell lineage commitment [GO:0002297] (biological process) Sources: GOC:add, ISBN:0781735149 Definition: The process in which a CD4-positive, alpha-beta T cell becomes committed to becoming a T-helper 2 cell, a CD4-positive, alpha-beta T cell specialized to promote immunological processes often associated with resistance to extracellular organisms such as helminths, enhanced production of particular antibody isotypes, and pathological conditions such as allergy. Also known as: T-helper 2 cell fate commitment, Th2 fate commitment Relationships: is a type of T-helper cell lineage commitment [GO:0002295]; is part of GO:0045064